positive regulation of proteolysis [GO:0045862] (biological process) Definition: Any process that activates or increases the frequency, rate or extent of the hydrolysis of a peptide bond or bonds within a protein. Relationships: is a type of GO:0030162; is a type of positive regulation of protein metabolic process [GO:0051247]; positively regulates proteolysis [GO:0006508] Sources: GOC:go_curators Also known as: positive regulation of peptidolysis, up regulation of proteolysis, up-regulation of proteolysis, upregulation of proteolysis, activation of proteolysis, stimulation of proteolysis Subtypes: positive regulation of peptidase activity [GO:0010952], positive regulation of protein processing [GO:0010954], GO:0051044, positive regulation of proteolysis involved in protein catabolic process [GO:1903052]